{
  "term_id": "GO:0005178",
  "gene_symbol": "TLN2",
  "gene_name": "Talin-2",
  "term_label": "integrin binding",
  "gene": "UniProtKB:Q9Y4G6"
}